{
  "gene_name": "BOS complex subunit NOMO1",
  "term_id": "UNKNOWN:0002",
  "gene_symbol": "NOMO1",
  "gene": "UniProtKB:Q15155",
  "term_label": "Unknown biological process"
}